glycerol-3-phosphate-glucose phosphotransferase activity [GO:0047327] (MF) Relationships: is a type of kinase activity [GO:0016301]; is a type of phosphotransferase activity, alcohol group as acceptor [GO:0016773] Also known as: sn-glycerol-3-phosphate:D-glucose 6-phosphotransferase activity Definition: Catalysis of the reaction: sn-glycerol 3-phosphate + D-glucose = D-glucose 6-phosphate + glycerol. Sources: EC:2.7.1.142, RHEA:21288